{
  "term_label": "cytokine receptor activity",
  "gene": "UniProtKB:P40189",
  "term_id": "GO:0004896",
  "gene_name": "Interleukin-6 receptor subunit beta",
  "gene_symbol": "IL6ST"
}